piRNA cluster binding [GO:1990470] (molecular function) Relationships: is_a sequence-specific double-stranded DNA binding [GO:1990837] Subtypes: piRNA uni-strand cluster binding [GO:1990471], piRNA dual-strand cluster binding [GO:1990472] References: PMID:24906153 Sources: GOC:bhm Definition: Binding to piRNA clusters, double-stranded DNA regions that give rise to PIWI-interacting RNAs (piRNAs). Note: An example of this is rhi in Drosophila melanogaster (Q7JXA8) in PMID:24906153 (inferred from direct assay).